positive regulation of tridecane biosynthetic process [GO:1900886] (biological process) Relationships: is a type of GO:1900884; is a type of positive regulation of alkane biosynthetic process [GO:1901579]; positively regulates tridecane biosynthetic process [GO:1900632] Sources: GOC:TermGenie, GOC:mengo_curators Definition: Any process that activates or increases the frequency, rate or extent of tridecane biosynthetic process. Also known as: positive regulation of tridecane anabolism, positive regulation of tridecane biosynthesis, positive regulation of tridecane formation, positive regulation of tridecane synthesis, up regulation of tridecane anabolism, up regulation of tridecane biosynthesis, up regulation of tridecane biosynthetic process, up regulation of tridecane formation, up regulation of tridecane synthesis, up-regulation of tridecane anabolism, up-regulation of tridecane biosynthesis, up-regulation of tridecane biosynthetic process, up-regulation of tridecane formation, up-regulation of tridecane synthesis, upregulation of tridecane anabolism, upregulation of tridecane biosynthesis, upregulation of tridecane biosynthetic process, upregulation of tridecane formation, upregulation of tridecane synthesis, activation of tridecane anabolism, activation of tridecane biosynthesis, activation of tridecane biosynthetic process, activation of tridecane formation, activation of tridecane synthesis